{
  "term_id": "GO:0005874",
  "term_label": "microtubule",
  "gene_symbol": "TUBB",
  "gene": "UniProtKB:P07437",
  "gene_name": "Tubulin beta chain"
}